protein transport within extracellular region [GO:0071693] (biological process) Relationships: is_a GO:0015031; is a type of establishment of protein localization to extracellular region [GO:0035592]; is_a protein localization to extracellular region [GO:0071692] Definition: The directed movement of proteins in the extracellular region, by means of some agent such as a transporter or pore. Sources: GOC:mah